concave side of sperm head [GO:0061830] (cellular component) Relationships: is_a cellular anatomical structure [GO:0110165]; is part of sperm head [GO:0061827] References: PMID:22332112, PMID:23403943, PMID:26990065 Definition: The concave part of the late spermatid head or spermatozoon head that forms the ventral portion of the head, particularly in some rodent species.